{
  "term_id": "GO:0006357",
  "gene_name": "Putative transcription factor SPT20 homolog-like 2",
  "term_label": "regulation of transcription by RNA polymerase II",
  "gene": "UniProtKB:P0C7V6",
  "gene_symbol": "SUPT20HL2"
}